{
  "term_label": "glucagon receptor activity",
  "term_id": "GO:0004967",
  "gene_symbol": "GLP1R",
  "gene": "UniProtKB:P43220",
  "gene_name": "Glucagon-like peptide 1 receptor"
}